{
  "gene_symbol": "PHF3",
  "gene_name": "PHD finger protein 3",
  "term_id": "UNKNOWN:0001",
  "gene": "UniProtKB:Q92576",
  "term_label": "Unknown molecular function"
}